{
  "term_label": "zinc ion binding",
  "gene_name": "Delta-aminolevulinic acid dehydratase",
  "gene": "UniProtKB:P13716",
  "term_id": "GO:0008270",
  "gene_symbol": "ALAD"
}